rolling circle DNA replication [GO:0070581] (biological process) Definition: A DNA-dependent DNA replication process in which a single-stranded DNA molecule is synthesized from a circular duplex template. Replication typically does not cease when one circumference has been replicated, but continues around the circumference several more times, producing a long single strand comprising multimers of the replicon. Relationships: is a type of DNA-templated DNA replication [GO:0006261] Also known as: rolling circle replication Sources: GOC:cb, GOC:mah, ISBN:0198506732